{
  "term_label": "cytokine-mediated signaling pathway",
  "gene_name": "PIK3R3 upstream open reading frame protein",
  "gene_symbol": "P3R3URF",
  "gene": "UniProtKB:A0A087WWA1",
  "term_id": "GO:0019221"
}